{
  "gene_symbol": "RAB3A",
  "term_id": "GO:0016079",
  "gene_name": "Ras-related protein Rab-3A",
  "term_label": "synaptic vesicle exocytosis",
  "gene": "UniProtKB:P20336"
}